{
  "term_label": "cell chemotaxis",
  "gene_symbol": "CXCR4",
  "gene": "UniProtKB:P61073",
  "gene_name": "C-X-C chemokine receptor type 4",
  "term_id": "GO:0060326"
}